1,2-diacyl-sn-glycero-3-phosphocholine metabolic process [GO:0006653] (biological process) Definition: The chemical reactions and pathways involving any 1,2-diacyl-sn-glycero-3-phosphocholine, the compounds most commonly designated lecithin. Relationships: is a type of phosphatidylcholine metabolic process [GO:0046470] Sources: ISBN:0198506732 Also known as: lecithin metabolic process, 1,2-diacyl-sn-glycero-3-phosphocholine metabolism